{
  "term_id": "GO:0005730",
  "term_label": "nucleolus",
  "gene": "UniProtKB:P62277",
  "gene_symbol": "RPS13",
  "gene_name": "Small ribosomal subunit protein uS15"
}